{
  "gene_name": "Serine_threonine-protein kinase tousled-like 2",
  "gene_symbol": "TLK2",
  "term_id": "GO:0048471",
  "gene": "UniProtKB:Q86UE8",
  "term_label": "perinuclear region of cytoplasm"
}